{
  "term_id": "UNKNOWN:0002",
  "gene": "UniProtKB:Q8N888",
  "gene_symbol": "BCORP1",
  "term_label": "Unknown biological process",
  "gene_name": "Putative BCoR-like protein 2"
}